{
  "gene": "UniProtKB:Q8IYS2",
  "term_label": "Unknown cellular component",
  "gene_name": "Uncharacterized protein KIAA2013",
  "term_id": "UNKNOWN:0003",
  "gene_symbol": "KIAA2013"
}